{
  "gene_name": "Beta-synuclein",
  "term_label": "axon terminus",
  "term_id": "GO:0043679",
  "gene": "UniProtKB:Q16143",
  "gene_symbol": "SNCB"
}